{
  "gene": "UniProtKB:O60641",
  "term_label": "phosphatidylinositol-4,5-bisphosphate binding",
  "gene_symbol": "SNAP91",
  "gene_name": "Clathrin coat assembly protein AP180",
  "term_id": "GO:0005546"
}